{
  "gene_symbol": "PDZD8",
  "term_id": "GO:0051560",
  "gene": "UniProtKB:Q8NEN9",
  "gene_name": "PDZ domain-containing protein 8",
  "term_label": "mitochondrial calcium ion homeostasis"
}